{
  "gene_name": "Bifunctional phosphoribosylaminoimidazole carboxylase_phosphoribosylaminoimidazole succinocarboxamide synthetase",
  "gene_symbol": "PAICS",
  "term_label": "'de novo' IMP biosynthetic process",
  "term_id": "GO:0006189",
  "gene": "UniProtKB:P22234"
}